{
  "term_label": "peptide antigen binding",
  "term_id": "GO:0042605",
  "gene_symbol": "HLA-DPB1",
  "gene_name": "HLA class II histocompatibility antigen, DP beta 1 chain",
  "gene": "UniProtKB:P04440"
}